adhesion of symbiont germination tube to host [GO:0075002] (biological process) Also known as: adhesion of symbiont germination tube to host during symbiotic interaction Definition: The attachment of a germination tube of the symbiont to its host via adhesion molecules. The host is defined as the larger of the organisms involved in a symbiotic interaction. Sources: GOC:pamgo_curators Relationships: is a type of adhesion of symbiont infection structure to host [GO:0075001] Note: Note that this term should not be used to annotate gene products of the host. It should only be used to annotate those gene products from the symbiont involved in this process.